plastid thylakoid [GO:0031976] (cellular component) Subtypes: chloroplast thylakoid [GO:0009534], cyanelle thylakoid [GO:0009843], prothylakoid [GO:0042649] Definition: Any thylakoid within a plastid. Sources: GOC:pz Relationships: is a type of thylakoid [GO:0009579]; is part of plastid [GO:0009536]